positive regulation of reciprocal meiotic recombination [GO:0010845] (biological process) Definition: Any process that increases the frequency, rate or extent of recombination during meiosis. Reciprocal meiotic recombination is the cell cycle process in which double strand breaks are formed and repaired through a double Holliday junction intermediate. Also known as: positive regulation of meiotic recombination Sources: GOC:dph, GOC:tb Relationships: is a type of GO:0010520; is a type of positive regulation of meiotic nuclear division [GO:0045836]; is a type of positive regulation of DNA recombination [GO:0045911]; positively regulates reciprocal meiotic recombination [GO:0007131] Subtypes: activation of reciprocal meiotic recombination [GO:0010846]